{
  "gene_name": "ATP-binding cassette sub-family C member 11",
  "term_id": "GO:0015721",
  "gene": "UniProtKB:Q96J66",
  "gene_symbol": "ABCC11",
  "term_label": "bile acid and bile salt transport"
}